{
  "gene": "UniProtKB:Q9BZC1",
  "gene_name": "CUGBP Elav-like family member 4",
  "term_label": "ribonucleoprotein complex",
  "term_id": "GO:1990904",
  "gene_symbol": "CELF4"
}